beta-zeacarotene biosynthetic process [GO:1901818] (biological process) Relationships: is a type of carotenoid biosynthetic process [GO:0016117]; is a type of carotene biosynthetic process [GO:0016120] References: PMID:3710717 Sources: GOC:TermGenie, GOC:yaf, UniPathway:UPA00805 Definition: The chemical reactions and pathways resulting in the formation of beta-zeacarotene. Also known as: beta-zeacarotene anabolism, beta-zeacarotene biosynthesis, beta-zeacarotene formation, beta-zeacarotene synthesis